{
  "term_id": "GO:0005856",
  "gene_name": "Protein STPG3",
  "term_label": "cytoskeleton",
  "gene": "UniProtKB:Q8N7X2",
  "gene_symbol": "STPG3"
}